{
  "term_id": "UNKNOWN:0003",
  "gene_symbol": "NUDT22",
  "gene": "UniProtKB:Q9BRQ3",
  "gene_name": "Uridine diphosphate glucose pyrophosphatase NUDT22",
  "term_label": "Unknown cellular component"
}